regulation of nucleotide-binding oligomerization domain containing 1 signaling pathway [GO:0070428] (biological process) Also known as: regulation of NOD1 signaling pathway, regulation of nucleotide-binding oligomerization domain containing 1 signalling pathway Subtypes: negative regulation of nucleotide-binding oligomerization domain containing 1 signaling pathway [GO:0070429], positive regulation of nucleotide-binding oligomerization domain containing 1 signaling pathway [GO:0070430] Definition: Any process that modulates the frequency, rate, or extent of the nucleotide-binding oligomerization domain containing 1 (NOD1) pathway. Relationships: is a type of GO:0070424; regulates GO:0070427 Sources: GOC:add